oleoyl-CoA ligase activity [GO:0090434] (molecular function) Also known as: oleoyl-CoA synthetase activity Definition: Catalysis of the reaction: ATP + oleic acid + CoA = AMP + diphosphate + oleoyl-CoA. Relationships: is_a long-chain fatty acid-CoA ligase activity [GO:0004467] References: PMID:18071249 Sources: GOC:al